regulation of protein K63-linked deubiquitination [GO:1903004] (biological process) Definition: Any process that modulates the frequency, rate or extent of protein K63-linked deubiquitination. References: PMID:22970133 Sources: GOC:PARL, GOC:TermGenie, GOC:bf, GO_REF:0000058 Relationships: is a type of regulation of protein deubiquitination [GO:0090085]; regulates GO:0070536 Subtypes: negative regulation of protein K63-linked deubiquitination [GO:1903005], positive regulation of protein K63-linked deubiquitination [GO:1903006]